{
  "term_label": "RNA polymerase II cis-regulatory region sequence-specific DNA binding",
  "gene": "UniProtKB:Q9Y458",
  "gene_name": "T-box transcription factor TBX22",
  "term_id": "GO:0000978",
  "gene_symbol": "TBX22"
}